pancreatic A cell differentiation [GO:0003310] (biological process) Definition: The process in which relatively unspecialized cells acquire specialized structural and functional features of a pancreatic A cell. A pancreatic A cell is a cell in the pancreas that secretes glucagon. References: PMID:11076772 Sources: GOC:dph Also known as: pancreatic alpha cell differentiation Relationships: is a type of enteroendocrine cell differentiation [GO:0035883]; is part of GO:0031018 Regulation: regulated by regulation of pancreatic A cell differentiation [GO:2000226]; negatively regulated by negative regulation of pancreatic A cell differentiation [GO:2000227]; positively regulated by positive regulation of pancreatic A cell differentiation [GO:2000228]